{
  "gene_name": "Zinc finger protein 22",
  "term_id": "GO:0010468",
  "term_label": "regulation of gene expression",
  "gene_symbol": "ZNF22",
  "gene": "UniProtKB:P17026"
}